Kdo2-lipid A biosynthetic process [GO:0036104] (biological process) Also known as: 3-deoxy-d-manno-octulosonic acid-lipid A biosynthesis, Kdo2-lipid A anabolism, Kdo2-lipid A biosynthesis, Kdo2-lipid A formation, Kdo2-lipid A synthesis Definition: The chemical reactions and pathways resulting in the formation of Kdo2-lipid A, a lipopolysaccharide (LPS) component. References: PMID:21106097 Sources: GOC:yaf Relationships: is_a GO:0008654; is a type of glycolipid biosynthetic process [GO:0009247]; is a type of dicarboxylic acid biosynthetic process [GO:0043650]; is a type of lipooligosaccharide biosynthetic process [GO:1901271]; is a type of fatty acid derivative biosynthetic process [GO:1901570]